limit dextrin alpha-1,6-maltotetraose-hydrolase activity [GO:0120549] (molecular function) Relationships: is a type of hydrolase activity, hydrolyzing O-glycosyl compounds [GO:0004553] Definition: Catalysis of the hydrolysis of (1->6)-alpha-D-glucosidic linkages to branches with degrees of polymerization of three or four glucose residues in limit dextrin. Sources: EC:3.2.1.196 Also known as: glycogen debranching enzyme